{
  "term_label": "endosomal transport",
  "gene_symbol": "ZFYVE9",
  "term_id": "GO:0016197",
  "gene_name": "Zinc finger FYVE domain-containing protein 9",
  "gene": "UniProtKB:O95405"
}